long descending thin limb development [GO:0072064] (biological process) Definition: The process whose specific outcome is the progression of the long descending thin limb over time, from its formation to the mature structure. The long descending thin limb is the descending thin limb of a long nephron that has a squamous epithelial morphology. The long descending limb starts in the inner stripe of the outer medulla and extends into the inner medulla. Subtypes: GO:0072269 Relationships: is a type of nephron epithelium development [GO:0072009]; is a type of GO:0072022; is part of long nephron development [GO:0072029] Sources: GOC:mtg_kidney_jan10